{
  "gene_symbol": "OR5B21",
  "term_label": "Unknown cellular component",
  "gene_name": "Olfactory receptor 5B21",
  "term_id": "UNKNOWN:0003",
  "gene": "UniProtKB:A6NL26"
}